superoxide dismutase activity [GO:0004784] (molecular function) Relationships: is a type of antioxidant activity [GO:0016209]; is a type of oxidoreductase activity, acting on superoxide radicals as acceptor [GO:0016721]; is part of removal of superoxide radicals [GO:0019430] References: PMID:15064408 Sources: EC:1.15.1.1, GOC:vw Regulation: regulated by regulation of superoxide dismutase activity [GO:1901668]; positively regulated by positive regulation of superoxide dismutase activity [GO:1901671] Also known as: superoxide:superoxide oxidoreductase activity, Cu-Zn superoxide dismutase activity, Mn, Fe superoxide dismutase, copper, zinc superoxide dismutase activity, ferrisuperoxide dismutase activity, iron superoxide dismutase activity, manganese superoxide dismutase activity, nickel superoxide dismutase activity, Cu,Zn-SOD, Fe-SOD, Mn-SOD, SOD, SOD-1, SOD-2, SOD-3, SOD-4, SODF, SODS, cuprein, cytocuprein, erythrocuprein, hemocuprein, hepatocuprein, iron superoxide oxidoreductase, manganese superoxide oxidoreductase, nickel superoxide oxidoreductase, superoxide dismutase I, superoxide dismutase II, zinc superoxide oxidoreductase Definition: Catalysis of the reaction: 2 superoxide + 2 H+ = O2 + hydrogen peroxide.